{
  "term_id": "UNKNOWN:0001",
  "term_label": "Unknown molecular function",
  "gene_name": "Opticin",
  "gene": "UniProtKB:Q9UBM4",
  "gene_symbol": "OPTC"
}